{
  "gene": "UniProtKB:Q75WM6",
  "term_id": "GO:0045910",
  "gene_name": "Testis-specific H1 histone",
  "term_label": "negative regulation of DNA recombination",
  "gene_symbol": "H1-7"
}